serotonin secretion by platelet [GO:0002554] (biological process) Relationships: is a type of serotonin secretion involved in inflammatory response [GO:0002442]; is a type of establishment of localization in cell [GO:0051649]; is a type of exocytic process [GO:0140029]; is part of platelet degranulation [GO:0002576] Also known as: serotonin release by platelet Sources: GOC:add, ISBN:0781735149 Definition: The regulated release of serotonin by a platelet or group of platelets.